{
  "gene_symbol": "GJA1",
  "gene_name": "Gap junction alpha-1 protein",
  "gene": "UniProtKB:P17302",
  "term_label": "heart development",
  "term_id": "GO:0007507"
}